{
  "gene_name": "Olfactory receptor 4M1",
  "term_label": "olfactory receptor activity",
  "term_id": "GO:0004984",
  "gene_symbol": "OR4M1",
  "gene": "UniProtKB:Q8NGD0"
}